positive regulation of hepatic stellate cell activation [GO:2000491] (biological process) Sources: GOC:obol Relationships: is a type of GO:0050867; is a type of regulation of hepatic stellate cell activation [GO:2000489]; positively regulates hepatic stellate cell activation [GO:0035733] Definition: Any process that activates or increases the frequency, rate or extent of hepatic stellate cell activation.